alpha-carotene biosynthetic process [GO:1901824] (biological process) Definition: The chemical reactions and pathways resulting in the formation of alpha-carotene. References: PMID:8837512 Sources: GOC:TermGenie, GOC:yaf, MetaCyc:PWY-5946, UniPathway:UPA00801 Also known as: delta-carotene anabolism, delta-carotene biosynthesis, delta-carotene biosynthetic process, delta-carotene formation, delta-carotene synthesis Relationships: is a type of carotenoid biosynthetic process [GO:0016117]; is a type of GO:0016120